{
  "term_id": "GO:0030020",
  "term_label": "extracellular matrix structural constituent conferring tensile strength",
  "gene_name": "Collagen alpha-2(I) chain",
  "gene": "UniProtKB:P08123",
  "gene_symbol": "COL1A2"
}